{
  "gene_symbol": "RNF34",
  "gene_name": "E3 ubiquitin-protein ligase RNF34",
  "term_label": "negative regulation of extrinsic apoptotic signaling pathway via death domain receptors",
  "term_id": "GO:1902042",
  "gene": "UniProtKB:Q969K3"
}